{
  "gene_symbol": "GGA1",
  "gene": "UniProtKB:Q9UJY5",
  "term_id": "GO:0006893",
  "gene_name": "ADP-ribosylation factor-binding protein GGA1",
  "term_label": "Golgi to plasma membrane transport"
}